{
  "gene_name": "Cancer_testis antigen 2",
  "term_label": "Unknown cellular component",
  "term_id": "UNKNOWN:0003",
  "gene": "UniProtKB:O75638",
  "gene_symbol": "CTAG2"
}